{
  "term_label": "protein processing involved in protein targeting to mitochondrion",
  "gene_symbol": "UQCRC1",
  "gene_name": "Cytochrome b-c1 complex subunit 1, mitochondrial",
  "gene": "UniProtKB:P31930",
  "term_id": "GO:0006627"
}